{
  "gene_symbol": "MAFK",
  "gene_name": "Transcription factor MafK",
  "term_id": "GO:0000978",
  "term_label": "RNA polymerase II cis-regulatory region sequence-specific DNA binding",
  "gene": "UniProtKB:O60675"
}